{
  "gene": "UniProtKB:Q8N485",
  "term_id": "GO:0097352",
  "gene_symbol": "LIX1",
  "gene_name": "Protein limb expression 1 homolog",
  "term_label": "autophagosome maturation"
}